chondroitin-sulfate-ABC endolyase activity [GO:0034000] (molecular function) Sources: EC:4.2.2.20 Definition: Catalysis of the endolytic cleavage of beta-1,4-galactosaminic bonds between N-acetylgalactosamine and either D-glucuronic acid or L-iduronic acid to produce a mixture of Delta4-unsaturated oligosaccharides of different sizes that are ultimately degraded to Delta4-unsaturated tetra- and disaccharides. Relationships: is a type of carbon-oxygen lyase activity, acting on polysaccharides [GO:0016837] Also known as: ChS ABC lyase activity, chondroitin ABC eliminase activity, chondroitin sulfate ABC lyase activity, chondroitinase ABC activity, chondroitinase activity, ChS ABC lyase I activity, chondroitin sulfate ABC endoeliminase activity, chondroitin sulfate ABC endolyase activity